nuclear DNA replication termination [GO:1902317] (biological process) Definition: Any DNA replication termination that is involved in nuclear cell cycle DNA replication. Relationships: is a type of cell cycle DNA replication termination [GO:1902294]; is part of nuclear DNA replication [GO:0033260] Also known as: DNA replication termination involved in DNA replication involved in S phase, DNA replication termination involved in DNA replication involved in S-phase, DNA replication termination involved in nuclear cell cycle DNA replication, DNA replication termination involved in DNA replication during S phase Sources: GOC:TermGenie, GOC:mtg_cell_cycle Subtypes: premeiotic DNA replication termination [GO:1902978], mitotic DNA replication termination [GO:1902979]